{
  "gene_name": "Heat shock factor protein 5",
  "gene_symbol": "HSF5",
  "term_id": "UNKNOWN:0002",
  "gene": "UniProtKB:Q4G112",
  "term_label": "Unknown biological process"
}